2-micrometer plasmid partitioning [GO:0030543] (biological process) Definition: The process in which copies of the 2-micrometer plasmid, found in fungi such as Saccharomyces, are distributed to daughter cells upon cell division. Relationships: is a type of plasmid partitioning [GO:0030541] Sources: GOC:mah